{
  "gene_name": "Vesicular glutamate transporter 1",
  "term_label": "neurotransmitter transmembrane transporter activity",
  "gene": "UniProtKB:Q9P2U7",
  "term_id": "GO:0005326",
  "gene_symbol": "SLC17A7"
}